{
  "term_label": "sperm principal piece",
  "term_id": "GO:0097228",
  "gene": "UniProtKB:Q15506",
  "gene_symbol": "SPA17",
  "gene_name": "Sperm surface protein Sp17"
}